protein digestion [GO:0044256] (biological process) Sources: GOC:go_curators Definition: The whole of the physical, chemical, and biochemical processes carried out by living organisms to break down ingested proteins into components that may be easily absorbed and directed into metabolism. Relationships: is_a digestion [GO:0007586]